{
  "gene_name": "Transient receptor potential cation channel subfamily M member 3",
  "term_label": "plasma membrane",
  "gene": "UniProtKB:Q9HCF6",
  "term_id": "GO:0005886",
  "gene_symbol": "TRPM3"
}